{
  "term_label": "neuron differentiation",
  "gene_symbol": "VAX2",
  "term_id": "GO:0030182",
  "gene_name": "Ventral anterior homeobox 2",
  "gene": "UniProtKB:Q9UIW0"
}